{
  "gene": "UniProtKB:Q8N8J6",
  "term_id": "GO:0000976",
  "term_label": "transcription cis-regulatory region binding",
  "gene_name": "Zinc finger protein 615",
  "gene_symbol": "ZNF615"
}